{
  "gene_name": "Lactotransferrin",
  "gene_symbol": "LTF",
  "term_id": "GO:0055037",
  "gene": "UniProtKB:P02788",
  "term_label": "recycling endosome"
}